{
  "gene_name": "BarH-like 2 homeobox protein",
  "gene": "UniProtKB:Q9NY43",
  "term_label": "RNA polymerase II transcription regulatory region sequence-specific DNA binding",
  "gene_symbol": "BARHL2",
  "term_id": "GO:0000977"
}